{
  "term_id": "UNKNOWN:0001",
  "term_label": "Unknown molecular function",
  "gene_name": "Serine_threonine-protein kinase 40",
  "gene_symbol": "STK40",
  "gene": "UniProtKB:Q8N2I9"
}